{
  "term_label": "very-low-density lipoprotein particle",
  "gene_name": "Apolipoprotein M",
  "gene": "UniProtKB:O95445",
  "gene_symbol": "APOM",
  "term_id": "GO:0034361"
}